{
  "gene": "UniProtKB:O43252",
  "gene_symbol": "PAPSS1",
  "term_id": "UNKNOWN:0003",
  "term_label": "Unknown cellular component",
  "gene_name": "Bifunctional 3'-phosphoadenosine 5'-phosphosulfate synthase 1"
}